negative regulation of cytokinesis [GO:0032466] (biological process) Definition: Any process that stops, prevents, or reduces the frequency, rate or extent of the division of the cytoplasm of a cell, and its separation into two daughter cells. Sources: GOC:mah Also known as: down regulation of cytokinesis, down-regulation of cytokinesis, downregulation of cytokinesis, inhibition of cytokinesis, negative regulation of cell cycle cytokinesis Relationships: is a type of negative regulation of cell cycle process [GO:0010948]; is a type of regulation of cytokinesis [GO:0032465]; is a type of negative regulation of cell division [GO:0051782]; negatively regulates GO:0000910 Subtypes: GO:1901892, negative regulation of mitotic cytokinesis [GO:1902413], negative regulation of cytokinesis, site selection [GO:2000075], GO:2000245, negative regulation of cytokinesis, actomyosin contractile ring assembly [GO:2000432]